proestrus [GO:0060208] (biological process) Note: Note that this term should not be used for direct annotation. If you are trying to make an annotation to x phase, it is likely that the correct annotation is 'regulation of x/y phase transition' or to a process which occurs during the reported phase. To capture the phase when a specific location or process is observed, the phase term can be used in an annotation extension (PMID:24885854) applied to a cellular component term (with the relation exists_during) or a biological process term (with the relation happens_during). Definition: The estrous cycle phase in which there is heightened follicular activity. Relationships: is a type of estrous cycle phase [GO:0060206] Sources: GOC:dph, ISBN:0721662544